{
  "term_id": "GO:0005737",
  "gene": "UniProtKB:Q9NSK0",
  "gene_name": "Kinesin light chain 4",
  "gene_symbol": "KLC4",
  "term_label": "cytoplasm"
}